{
  "term_id": "GO:0009898",
  "term_label": "cytoplasmic side of plasma membrane",
  "gene": "UniProtKB:Q9BY43",
  "gene_name": "Charged multivesicular body protein 4a",
  "gene_symbol": "CHMP4A"
}